{
  "gene_name": "Putative taste receptor type 2 member 36",
  "term_label": "membrane",
  "gene": "UniProtKB:P0DTE0",
  "term_id": "GO:0016020",
  "gene_symbol": "TAS2R36"
}